{
  "gene_symbol": "BAG5",
  "term_id": "GO:0005829",
  "term_label": "cytosol",
  "gene": "UniProtKB:Q9UL15",
  "gene_name": "BAG family molecular chaperone regulator 5"
}